hydroquinone:oxygen oxidoreductase activity [GO:0052716] (molecular function) Definition: Catalysis of the reaction: 4 hydroquinone + O2 = 4 benzosemiquinone + 4 H2O. Sources: EC:1.10.3.2 Also known as: benzenediol:oxygen oxidoreductase activity, laccase reaction, p-diphenol:oxygen oxidoreductase activity Relationships: is a type of oxidoreductase activity, acting on diphenols and related substances as donors, oxygen as acceptor [GO:0016682]